cellular response to high light intensity [GO:0071486] (biological process) Relationships: is a type of response to high light intensity [GO:0009644]; is a type of GO:0071484 Definition: Any process that results in a change in state or activity of a cell (in terms of movement, secretion, enzyme production, gene expression, etc.) as a result of a high light intensity stimulus. Sources: GOC:mah